amino acid import across plasma membrane [GO:0089718] (BP) Regulation: regulated by regulation of amino acid import across plasma membrane [GO:0010958] Subtypes: D-aspartate import across plasma membrane [GO:0070779], GO:0097638, L-lysine import across plasma membrane [GO:0097639], L-ornithine import across plasma membrane [GO:0097640], L-glutamate import across plasma membrane [GO:0098712], GO:0098718, L-aspartate import across plasma membrane [GO:0140009], 5-aminolevulinic acid import across plasma membrane [GO:0140484], L-phenylalanine import across plasma membrane [GO:0140925], methionine import across plasma membrane [GO:1903692], L-leucine import across plasma membrane [GO:1903801], L-glutamine import across plasma membrane [GO:1903803], glycine import across plasma membrane [GO:1903804], L-valine import across plasma membrane [GO:1903805], L-isoleucine import across plasma membrane [GO:1903806], L-threonine import across plasma membrane [GO:1903807], L-tyrosine import across plasma membrane [GO:1903808], GO:1903810, GO:1903811, L-tryptophan import across plasma membrane [GO:1904272], GO:1904273, proline import across plasma membrane [GO:1905647] References: PMID:8195186 Sources: GOC:krc Relationships: is a type of amino acid transmembrane transport [GO:0003333]; is a type of import across plasma membrane [GO:0098739] Also known as: L-amino acid import, amino acid transmembrane import, amino acid import into cell, L-amino acid uptake Definition: The directed movement of an amino acid from outside of a cell, across the plasma membrane and into the cytosol.